{
  "gene_symbol": "BCL2L15",
  "gene": "UniProtKB:Q5TBC7",
  "gene_name": "Bcl-2-like protein 15",
  "term_label": "Unknown biological process",
  "term_id": "UNKNOWN:0002"
}